{
  "gene": "UniProtKB:Q86WD7",
  "gene_symbol": "SERPINA9",
  "term_label": "extracellular space",
  "gene_name": "Serpin A9",
  "term_id": "GO:0005615"
}